left ventricular compact myocardium morphogenesis [GO:0003224] (biological process) Definition: The process in which the anatomical structures of cardiac left ventricular compact myocardium are generated and organized. Sources: GOC:mtg_heart Relationships: is a type of GO:0003220; is a type of GO:0003223